GMP reductase activity [GO:0003920] (molecular function) Sources: EC:1.7.1.7, RHEA:17185 Definition: Catalysis of the reaction: IMP + NADP+ + NH4 = GMP + 2 H+ + NADPH. Also known as: NADPH2:guanosine-5'-phosphate oxidoreductase (deaminating), NADPH:GMP oxidoreductase (deaminating) activity, NADPH:guanosine-5'-phosphate oxidoreductase (deaminating) activity, guanosine 5'-monophosphate oxidoreductase activity, guanosine 5'-monophosphate reductase activity, guanosine 5'-phosphate reductase activity, guanosine monophosphate reductase activity, guanylate reductase activity, inosine-5'-phosphate:NADP+ oxidoreductase (aminating) Relationships: is a type of oxidoreductase activity, acting on other nitrogenous compounds as donors, with NAD or NADP as acceptor [GO:0046857]